{
  "gene_symbol": "FBXO40",
  "gene_name": "F-box only protein 40",
  "term_label": "cytoplasm",
  "term_id": "GO:0005737",
  "gene": "UniProtKB:Q9UH90"
}